{
  "term_id": "GO:0003934",
  "gene_name": "GTP cyclohydrolase 1",
  "gene": "UniProtKB:P30793",
  "gene_symbol": "GCH1",
  "term_label": "GTP cyclohydrolase I activity"
}